{
  "gene_symbol": "HHLA1",
  "gene": "UniProtKB:C9JL84",
  "gene_name": "HERV-H LTR-associating protein 1",
  "term_label": "Unknown molecular function",
  "term_id": "UNKNOWN:0001"
}